vesicle targeting, plasma membrane to endosome [GO:0048201] (biological process) Relationships: is a type of vesicle targeting [GO:0006903] Also known as: plasma membrane to endosome targeting Definition: The process in which vesicles formed at the plasma membrane are directed to specific destinations in endosome membranes, mediated by molecules at the vesicle membrane and target membrane surfaces. References: PMID:10219233 Sources: GOC:jid, GOC:mah, ISBN:0716731363